{
  "gene_name": "PRO2179",
  "term_label": "Unknown molecular function",
  "term_id": "UNKNOWN:0001",
  "gene": "UniProtKB:Q9H3A6",
  "gene_symbol": "Q9H3A6"
}